{
  "term_id": "GO:0005737",
  "gene_symbol": "AK9",
  "gene_name": "Adenylate kinase 9",
  "gene": "UniProtKB:Q5TCS8",
  "term_label": "cytoplasm"
}